{
  "gene_symbol": "DLG4",
  "gene": "UniProtKB:P78352",
  "term_label": "nervous system development",
  "term_id": "GO:0007399",
  "gene_name": "Disks large homolog 4"
}